negative regulation of gonadotropin secretion [GO:0032277] (biological process) Definition: Any process that stops, prevents, or reduces the frequency, rate or extent of the regulated release of a gonadotropin. Sources: GOC:mah Also known as: down regulation of gonadotropin secretion, down-regulation of gonadotropin secretion, downregulation of gonadotropin secretion, negative regulation of gonadotrophin secretion, inhibition of gonadotropin secretion Relationships: is a type of regulation of gonadotropin secretion [GO:0032276]; is a type of negative regulation of hormone secretion [GO:0046888]; is a type of GO:0051241; negatively regulates gonadotropin secretion [GO:0032274] Subtypes: negative regulation of luteinizing hormone secretion [GO:0033685], negative regulation of follicle-stimulating hormone secretion [GO:0046882]